{
  "term_id": "GO:0000956",
  "gene": "UniProtKB:Q9NQT5",
  "gene_symbol": "EXOSC3",
  "term_label": "nuclear-transcribed mRNA catabolic process",
  "gene_name": "Exosome complex component RRP40"
}